{
  "gene_name": "3-oxoacyl-[acyl-carrier-protein] synthase, mitochondrial",
  "term_id": "GO:0004315",
  "gene": "UniProtKB:Q9NWU1",
  "gene_symbol": "OXSM",
  "term_label": "3-oxoacyl-[acyl-carrier-protein] synthase activity"
}